{
  "term_id": "GO:0002009",
  "gene_name": "Keratin, type I cytoskeletal 14",
  "gene_symbol": "KRT14",
  "term_label": "morphogenesis of an epithelium",
  "gene": "UniProtKB:P02533"
}